anthranilate phosphoribosyltransferase activity [GO:0004048] (molecular function) Relationships: is a type of pentosyltransferase activity [GO:0016763] Definition: Catalysis of the reaction: N-(5-phospho-beta-D-ribosyl)anthranilate + diphosphate = 5-phospho-alpha-D-ribose 1-diphosphate + anthranilate. Sources: EC:2.4.2.18, RHEA:11768 Also known as: N-(5-phospho-D-ribosyl)-anthranilate:diphosphate phospho-alpha-D-ribosyltransferase activity, PRT, anthranilate 5-phosphoribosylpyrophosphate phosphoribosyltransferase activity, anthranilate phosphoribosylpyrophosphate phosphoribosyltransferase activity, anthranilate-PP-ribose-P phosphoribosyltransferase activity, phosphoribosyl-anthranilate diphosphorylase activity, phosphoribosyl-anthranilate pyrophosphorylase activity, phosphoribosylanthranilate pyrophosphorylase activity, phosphoribosylanthranilate transferase activity